{
  "term_label": "action potential",
  "gene_symbol": "KCNC2",
  "gene": "UniProtKB:Q96PR1",
  "term_id": "GO:0001508",
  "gene_name": "Potassium voltage-gated channel subfamily C member 2"
}